{
  "gene_symbol": "ABHD13",
  "term_label": "plasma membrane",
  "term_id": "GO:0005886",
  "gene": "UniProtKB:Q7L211",
  "gene_name": "Protein ABHD13"
}